{
  "term_id": "UNKNOWN:0001",
  "gene_name": "Mitochondrial fission process protein 1",
  "gene": "UniProtKB:Q9UDX5",
  "gene_symbol": "MTFP1",
  "term_label": "Unknown molecular function"
}